{
  "term_label": "postsynaptic density",
  "gene_symbol": "PPP1R9A",
  "term_id": "GO:0014069",
  "gene": "UniProtKB:Q9ULJ8",
  "gene_name": "Neurabin-1"
}